type 1 angiotensin receptor binding [GO:0031702] (molecular function) Also known as: AT1 receptor binding, type 1 angiotensin receptor ligand Relationships: is a type of GO:0031701 Definition: Binding to a type 1 angiotensin receptor. Sources: GOC:mah, GOC:nln